{
  "gene_name": "Putative histone H2B type 2-D",
  "gene_symbol": "H2BC19P",
  "gene": "UniProtKB:Q6DRA6",
  "term_label": "DNA binding",
  "term_id": "GO:0003677"
}